{
  "term_id": "GO:0005634",
  "gene": "UniProtKB:Q09666",
  "gene_symbol": "AHNAK",
  "gene_name": "Neuroblast differentiation-associated protein AHNAK",
  "term_label": "nucleus"
}